{
  "term_id": "GO:0045116",
  "gene_name": "NEDD8-activating enzyme E1 catalytic subunit",
  "gene_symbol": "UBA3",
  "gene": "UniProtKB:Q8TBC4",
  "term_label": "protein neddylation"
}